{
  "term_label": "contractile ring",
  "gene_symbol": "ALKBH4",
  "term_id": "GO:0070938",
  "gene_name": "Alpha-ketoglutarate-dependent dioxygenase alkB homolog 4",
  "gene": "UniProtKB:Q9NXW9"
}